{
  "gene": "UniProtKB:P43358",
  "gene_name": "Melanoma-associated antigen 4",
  "term_label": "nucleus",
  "gene_symbol": "MAGEA4",
  "term_id": "GO:0005634"
}